{
  "gene_name": "Exosome RNA helicase MTR4",
  "term_id": "GO:0031499",
  "gene": "UniProtKB:P42285",
  "term_label": "TRAMP complex",
  "gene_symbol": "MTREX"
}